{
  "term_label": "transmembrane transporter activity",
  "gene_symbol": "TMEM184A",
  "gene_name": "Transmembrane protein 184A",
  "term_id": "GO:0022857",
  "gene": "UniProtKB:Q6ZMB5"
}